{
  "gene_name": "Putative synaptotagmin-14-like protein",
  "gene": "UniProtKB:Q58G82",
  "gene_symbol": "SYT14P1",
  "term_label": "Unknown cellular component",
  "term_id": "UNKNOWN:0003"
}